follicle-stimulating hormone receptor activity [GO:0004963] (molecular function) Definition: Combining with follicle-stimulating hormone to initiate a change in cell activity. Relationships: is_a protein-hormone receptor activity [GO:0016500]; is part of follicle-stimulating hormone signaling pathway [GO:0042699] Sources: GOC:mah Also known as: FSH receptor activity, follicle stimulating hormone receptor activity